hemi-methylated DNA-binding [GO:0044729] (molecular function) Relationships: is a type of double-stranded DNA binding [GO:0003690] Definition: Binding to double-stranded hemi-methylated DNA at replication foci (one strand methylated, while the other strand is unmethylated). Methylation of cytosine or adenine in DNA is an important mechanism for establishing stable heritable epigenetic marks. References: PMID:18772889 Sources: GOC:imk, GOC:sp Also known as: double-stranded hemi-methylated DNA binding